{
  "gene_name": "Gap junction alpha-9 protein",
  "term_label": "cell-cell signaling",
  "term_id": "GO:0007267",
  "gene": "UniProtKB:P57773",
  "gene_symbol": "GJA9"
}